{
  "gene_symbol": "ZNF646",
  "gene": "UniProtKB:O15015",
  "gene_name": "Zinc finger protein 646",
  "term_id": "GO:0006355",
  "term_label": "regulation of DNA-templated transcription"
}